{
  "term_id": "UNKNOWN:0001",
  "term_label": "Unknown molecular function",
  "gene_symbol": "CSPG4",
  "gene_name": "Chondroitin sulfate proteoglycan 4",
  "gene": "UniProtKB:Q6UVK1"
}